viral head-tail joining [GO:0098005] (biological process) Also known as: virus head-tail joining, phage head tail joining Sources: GOC:bm Relationships: is a type of GO:0016032; is part of GO:0019068 Definition: Process by which virus heads and tails are attached to each other.